{
  "term_label": "endoplasmic reticulum",
  "gene": "UniProtKB:Q9UIJ5",
  "gene_symbol": "ZDHHC2",
  "gene_name": "Palmitoyltransferase ZDHHC2",
  "term_id": "GO:0005783"
}